polarity specification of proximal/distal axis [GO:0010085] (biological process) Relationships: is a type of specification of axis polarity [GO:0065001]; is part of proximal/distal axis specification [GO:0009946] Sources: GOC:tb Definition: Any process resulting in the establishment of polarity along the proximal/distal axis.